{
  "gene": "UniProtKB:P35453",
  "gene_symbol": "HOXD13",
  "gene_name": "Homeobox protein Hox-D13",
  "term_label": "DNA-binding transcription factor activity, RNA polymerase II-specific",
  "term_id": "GO:0000981"
}